glutathione hydrolase activity [GO:0036374] (molecular function) Sources: EC:3.4.19.13, GOC:imk Definition: Catalysis of the reaction: glutathione + H2O = L-cysteinylglycine + L-glutamate. Relationships: is a type of omega peptidase activity [GO:0008242]; is a type of GO:0070003 Also known as: gamma-glutamyltranspeptidase activity, glutathionase activity